epiblast cell-extraembryonic ectoderm cell signaling [GO:0060802] (biological process) Relationships: is a type of cell-cell signaling [GO:0007267] Definition: Any process that mediates the transfer of information from an epiblast cell to an extraembryonic ectoderm cell. References: PMID:14511481, PMID:31391456 Sources: GOC:dph, GOC:tb